{
  "gene_name": "Protein arginine N-methyltransferase 3",
  "gene": "UniProtKB:O60678",
  "term_id": "GO:0005634",
  "term_label": "nucleus",
  "gene_symbol": "PRMT3"
}